{
  "term_id": "GO:0016477",
  "term_label": "cell migration",
  "gene_symbol": "CTNNA3",
  "gene": "UniProtKB:Q9UI47",
  "gene_name": "Catenin alpha-3"
}